{
  "term_id": "GO:0030855",
  "gene_name": "Keratin, type I cytoskeletal 23",
  "gene": "UniProtKB:Q9C075",
  "term_label": "epithelial cell differentiation",
  "gene_symbol": "KRT23"
}